{
  "gene_name": "Probable ATP-dependent RNA helicase DDX6",
  "term_label": "mRNA binding",
  "term_id": "GO:0003729",
  "gene_symbol": "DDX6",
  "gene": "UniProtKB:P26196"
}